{
  "gene_symbol": "GPX1",
  "gene": "UniProtKB:P07203",
  "term_id": "GO:0004602",
  "gene_name": "Glutathione peroxidase 1",
  "term_label": "glutathione peroxidase activity"
}